2-hydroxyglutaryl-CoA dehydratase activity [GO:0043717] (molecular function) Sources: MetaCyc:RXN-1083 Definition: Catalysis of the reaction: (R)-2-hydroxyglutaryl-CoA = H2O + glutaconyl-CoA. Relationships: is a type of GO:0016836 Also known as: (R)-2-hydroxyglutaryl-CoA dehydratase activity